ascending thin limb development [GO:0072021] (biological process) Relationships: is a type of nephron tubule development [GO:0072080]; is part of loop of Henle development [GO:0072070] Subtypes: GO:0072218 Definition: The process whose specific outcome is the progression of an ascending thin limb over time, from its formation to the mature structure. The ascending thin limb is a segment of a nephron tubule lying in the inner medulla that is permeable to ions but not to water and has a simple epithelium; active transepithelial solute transport is absent. Sources: GOC:mtg_kidney_jan10